{
  "gene": "UniProtKB:P28347",
  "gene_symbol": "TEAD1",
  "gene_name": "Transcriptional enhancer factor TEF-1",
  "term_id": "GO:0005667",
  "term_label": "transcription regulator complex"
}